[pyruvate dehydrogenase (acetyl-transferring)]-phosphatase activity [GO:0004741] (molecular function) Definition: Catalysis of the reaction: O-phospho-L-seryl-[pyruvate dehydrogenase E1 alpha subunit] + H2O = L-seryl-[pyruvate dehydrogenase E1 alpha subunit] + phosphate. Sources: EC:3.1.3.43 Also known as: [pyruvate dehydrogenase (lipoamide)] phosphatase activity, [pyruvate dehydrogenase (lipoamide)] phosphatase, intrinsic catalyst activity, pyruvate dehydrogenase (lipoamide) phosphatase activity Relationships: is a type of protein serine/threonine phosphatase activity [GO:0004722]